{
  "term_label": "phospholipase A1 activity",
  "term_id": "GO:0008970",
  "gene": "UniProtKB:P11150",
  "gene_symbol": "LIPC",
  "gene_name": "Hepatic triacylglycerol lipase"
}